meiotic DNA repair synthesis [GO:0000711] (biological process) Definition: During meiosis, the synthesis of DNA proceeding from the broken 3' single-strand DNA end that uses the homologous intact duplex as the template. References: PMID:9334324 Sources: GOC:elh Relationships: is a type of DNA synthesis involved in DNA repair [GO:0000731]; is a type of meiosis I cell cycle process [GO:0061982] Subtypes: meiotic DNA repair synthesis involved in reciprocal meiotic recombination [GO:0010778], meiotic DNA repair synthesis involved in meiotic gene conversion [GO:0010779]